{
  "gene_symbol": "PDE11A",
  "term_id": "GO:0047555",
  "gene_name": "Dual 3',5'-cyclic-AMP and -GMP phosphodiesterase 11A",
  "gene": "UniProtKB:Q9HCR9",
  "term_label": "3',5'-cyclic-GMP phosphodiesterase activity"
}